insecticide metabolic process [GO:0017143] (biological process) Definition: The chemical reactions and pathways involving insecticides, chemicals used to kill insects. Subtypes: 1,1,1-trichloro-2,2-bis-(4-chlorophenyl)ethane metabolic process [GO:0018977], GO:0046701 Relationships: is a type of xenobiotic metabolic process [GO:0006805]; is a type of toxin metabolic process [GO:0009404]; is part of response to insecticide [GO:0017085] Sources: GOC:ai Also known as: insecticide metabolism